protein complex involved in cell-matrix adhesion [GO:0098637] (cellular component) Subtypes: collagen type XVII trimer [GO:0030937], tenascin complex [GO:0090733], EMILIN complex [GO:1990971], multimerin complex [GO:1990972] Definition: Any protein complex that is capable of carrying out some part of the process of cell-matrix adhesion. Sources: GOC:dos Relationships: is a type of protein complex involved in cell adhesion [GO:0098636]